{
  "term_id": "GO:0006955",
  "gene_symbol": "CD1A",
  "term_label": "immune response",
  "gene_name": "T-cell surface glycoprotein CD1a",
  "gene": "UniProtKB:P06126"
}